regulation of jasmonic acid biosynthetic process [GO:0080141] (biological process) Sources: GOC:dhl Relationships: is a type of regulation of fatty acid biosynthetic process [GO:0042304]; is a type of regulation of jasmonic acid metabolic process [GO:0080140]; regulates jasmonic acid biosynthetic process [GO:0009695] Definition: Any process that modulates the frequency, rate or extent of the chemical reactions and pathways resulting in the formation of jasmonic acid.